collagen type I trimer [GO:0005584] (cellular component) Definition: A collagen trimer containing alpha(I) chains. The most common form of type I collagen is a heterotrimer containing two alpha1(I) chains and one alpha2(I) chain; homotrimers containing three alpha1(I) chains are also found. Type I collagen triple helices associate to form banded fibrils. References: PMID:21421911 Relationships: is a type of GO:0005583